PAS complex [GO:0070772] (cellular component) Definition: A phosphatidylinositol kinase complex that contains a phosphatidylinositol-3-phosphate 5-kinase subunit (Fab1p in yeast; PIKFYVE in mammals), a kinase activator, and a phosphatase, and may also contain additional proteins; it is involved in regulating the synthesis and turnover of phosphatidylinositol 3,5-bisphosphate. In mammals the complex is composed of PIKFYVE, FIG4 and VAC14. In yeast it is composed of Atg18p, Fig4p, Fab1p, Vac14p and Vac7p. Relationships: is a type of GO:0061695; is_a GO:0098796; BFO_0000050 vacuolar membrane [GO:0005774] Also known as: autophagy-specific phosphatidylinositol 3-kinase complex References: PMID:18950639, PMID:19037259, PMID:19158662